{
  "term_id": "GO:1904315",
  "gene_symbol": "HTR3D",
  "term_label": "transmitter-gated monoatomic ion channel activity involved in regulation of postsynaptic membrane potential",
  "gene_name": "5-hydroxytryptamine receptor 3D",
  "gene": "UniProtKB:Q70Z44"
}